{
  "gene": "UniProtKB:Q6P1K1",
  "term_id": "GO:0015232",
  "gene_symbol": "SLC48A1",
  "term_label": "heme transmembrane transporter activity",
  "gene_name": "Heme transporter HRG1"
}